{
  "gene_symbol": "GCNT1",
  "term_label": "Unknown biological process",
  "gene_name": "Beta-1,3-galactosyl-O-glycosyl-glycoprotein beta-1,6-N-acetylglucosaminyltransferase",
  "term_id": "UNKNOWN:0002",
  "gene": "UniProtKB:Q02742"
}